cellular response to L-canavanine [GO:0036280] (biological process) Definition: Any process that results in a change in state or activity of a cell (in terms of movement, secretion, enzyme production, gene expression, etc.) as a result of a L-canavanine stimulus. L-canavanine is L-homoserine substituted at oxygen with a guanidino (carbamimidamido) group. Sources: GOC:al Relationships: is a type of cellular response to amino acid stimulus [GO:0071230]; is a type of response to L-canavanine [GO:1901354]; is a type of GO:1901699; is a type of cellular response to oxygen-containing compound [GO:1901701]